{
  "gene": "UniProtKB:Q13129",
  "term_label": "nucleus",
  "term_id": "GO:0005634",
  "gene_symbol": "RLF",
  "gene_name": "Zinc finger protein Rlf"
}